{
  "gene_symbol": "IGF1R",
  "term_id": "GO:0046328",
  "gene": "UniProtKB:P08069",
  "term_label": "regulation of JNK cascade",
  "gene_name": "Insulin-like growth factor 1 receptor"
}